{
  "term_label": "immune response",
  "gene_symbol": "C17orf99",
  "term_id": "GO:0006955",
  "gene": "UniProtKB:Q6UX52",
  "gene_name": "Protein IL-40"
}